delamination involved in gastrulation with mouth forming second [GO:0055112] (biological process) Definition: The splitting or migration of one epithelial sheet into two involved in the process of deuterostomic gastrulation. Sources: ISBN:0878932437 Relationships: is a type of delamination [GO:0060232]; is part of gastrulation with mouth forming second [GO:0001702]